negative regulation of interleukin-32 production [GO:0150190] (biological process) Relationships: is a type of negative regulation of cytokine production [GO:0001818]; is a type of regulation of interleukin-32 production [GO:0150189]; RO_0002212 GO:0072637 Also known as: negative regulation of interleukin-32 biosynthetic process, negative regulation of interleukin-32 secretion Definition: Any process that stops, prevents or reduces the frequency, rate or extent of interleukin-32 production. References: PMID:23729669 Sources: GOC:aruk